{
  "gene_name": "Centromere protein I",
  "gene_symbol": "CENPI",
  "term_id": "GO:0034080",
  "term_label": "CENP-A containing chromatin assembly",
  "gene": "UniProtKB:Q92674"
}